alpha-1,3-galactosyltransferase activity [GO:0001962] (molecular function) Also known as: isoglobotriaosylceramide synthase Relationships: is_a galactosyltransferase activity [GO:0008378] References: PMID:10854427 Sources: GOC:hjd Definition: Catalysis of the transfer of a galactose residue from a donor molecule, such as GDP-galactose or UDP-galactose, to an oligosaccharide, forming an alpha-(1->3) linkage.